alditol biosynthetic process [GO:0019401] (biological process) Relationships: is a type of carbohydrate biosynthetic process [GO:0016051]; is a type of GO:0046173 Definition: The chemical reactions and pathways resulting in the formation of alditols, any polyhydric alcohol derived from the acyclic form of a monosaccharide by reduction of its aldehyde or keto group to an alcoholic group. Sources: ISBN:0198506732 Subtypes: glycerol biosynthetic process [GO:0006114], GO:0019406, GO:0019526, glucosylglycerol biosynthetic process [GO:0051473] Also known as: alditol anabolism, alditol biosynthesis, alditol formation, alditol synthesis